{
  "gene": "UniProtKB:Q9HCK8",
  "term_label": "nucleus",
  "gene_name": "Chromodomain-helicase-DNA-binding protein 8",
  "term_id": "GO:0005634",
  "gene_symbol": "CHD8"
}